detection of chemical stimulus involved in sensory perception of bitter taste [GO:0001580] (biological process) Definition: The series of events required for a bitter taste stimulus to be received and converted to a molecular signal. Sources: GOC:go_curators Relationships: is a type of detection of chemical stimulus involved in sensory perception of taste [GO:0050912]; is part of GO:0050913 Also known as: bitter taste detection, perception of bitter taste, detection of chemical stimulus, perception of bitter taste, sensory transduction of chemical stimulus, sensory detection of bitter taste, sensory detection of chemical stimulus during perception of bitter taste, sensory transduction of bitter taste, sensory transduction of chemical stimulus during perception of bitter taste